cytoskeletal calyx [GO:0033150] (cellular component) Definition: A large cytoskeletal structure located at the posterior end of the perinuclear theca of a mammalian sperm head. The nucleus is tightly associated with the calyx, which contains calicin and basic cylicin proteins. References: PMID:12243744, PMID:9184090 Relationships: is a type of cellular anatomical structure [GO:0110165]; is part of perinuclear theca [GO:0033011]